{
  "term_label": "Unknown cellular component",
  "term_id": "UNKNOWN:0003",
  "gene_symbol": "FAM185A",
  "gene": "UniProtKB:Q8N0U4",
  "gene_name": "Protein FAM185A"
}